{
  "term_id": "GO:0006749",
  "gene_name": "glutathione transferase",
  "gene": "UniProtKB:A0A1W2PRG0",
  "gene_symbol": "GSTTP2",
  "term_label": "glutathione metabolic process"
}